{
  "gene_name": "Protein disulfide isomerase CRELD2",
  "term_label": "extracellular matrix",
  "term_id": "GO:0031012",
  "gene_symbol": "CRELD2",
  "gene": "UniProtKB:Q6UXH1"
}